{
  "gene_name": "Putative endogenous retrovirus group K member 11-1 Env polyprotein",
  "gene_symbol": "ERVK11-1",
  "gene": "UniProtKB:P61568",
  "term_id": "UNKNOWN:0001",
  "term_label": "Unknown molecular function"
}